{
  "gene": "UniProtKB:P07900",
  "term_label": "protein-containing complex",
  "term_id": "GO:0032991",
  "gene_symbol": "HSP90AA1",
  "gene_name": "Heat shock protein HSP 90-alpha"
}